{
  "term_id": "GO:0043410",
  "gene_symbol": "ADRA1A",
  "term_label": "positive regulation of MAPK cascade",
  "gene_name": "Alpha-1A adrenergic receptor",
  "gene": "UniProtKB:P35348"
}